neuropeptide F receptor binding [GO:0071859] (molecular function) Relationships: is a type of neuropeptide receptor binding [GO:0071855] Definition: Binding to a neuropeptide F receptor. Sources: GOC:kmv, GOC:mah